L-phenylalanine metabolic process [GO:0006558] (biological process) Sources: GOC:jsg, GOC:mah Also known as: phenylalanine metabolic process, phenylalanine metabolism, L-phenylalanine metabolism Relationships: is a type of aromatic amino acid metabolic process [GO:0009072]; is a type of L-amino acid metabolic process [GO:0170033]; is a type of proteinogenic amino acid metabolic process [GO:0170039] Subtypes: L-phenylalanine catabolic process [GO:0006559], L-phenylalanine biosynthetic process [GO:0009094] Definition: The chemical reactions and pathways involving L-phenylalanine, the L-enantiomer of 2-amino-3-phenylpropanoic acid, i.e. (2S)-2-amino-3-phenylpropanoic acid.